ribonucleoside catabolic process [GO:0042454] (biological process) Relationships: is a type of ribonucleoside metabolic process [GO:0009119]; is a type of nucleoside catabolic process [GO:0009164] Sources: GOC:jl Definition: The chemical reactions and pathways resulting in the breakdown of any ribonucleoside, a nucleoside in which purine or pyrimidine base is linked to a ribose (beta-D-ribofuranose) molecule. Also known as: ribonucleoside breakdown, ribonucleoside catabolism, ribonucleoside degradation Subtypes: purine ribonucleoside catabolic process [GO:0046130], pyrimidine ribonucleoside catabolic process [GO:0046133]